{
  "gene": "UniProtKB:Q8N7J2",
  "term_id": "GO:0005546",
  "gene_symbol": "AMER2",
  "term_label": "phosphatidylinositol-4,5-bisphosphate binding",
  "gene_name": "APC membrane recruitment protein 2"
}